{
  "term_id": "GO:0005794",
  "gene": "UniProtKB:Q9NWB7",
  "term_label": "Golgi apparatus",
  "gene_symbol": "IFT57",
  "gene_name": "Intraflagellar transport protein 57 homolog"
}